{
  "gene": "UniProtKB:Q96MT8",
  "gene_symbol": "CEP63",
  "term_label": "Unknown molecular function",
  "term_id": "UNKNOWN:0001",
  "gene_name": "Centrosomal protein of 63 kDa"
}